{
  "term_label": "Unknown cellular component",
  "gene": "UniProtKB:P0DM63",
  "gene_name": "Nuclear pore complex-interacting protein family member A8",
  "term_id": "UNKNOWN:0003",
  "gene_symbol": "NPIPA8"
}